{
  "term_label": "defense response to Gram-negative bacterium",
  "gene_name": "Ribonuclease 7",
  "gene": "UniProtKB:Q9H1E1",
  "term_id": "GO:0050829",
  "gene_symbol": "RNASE7"
}